{
  "gene_name": "Spermatogenesis- and oogenesis-specific basic helix-loop-helix-containing protein 2",
  "term_label": "DNA-binding transcription factor activity, RNA polymerase II-specific",
  "gene_symbol": "SOHLH2",
  "gene": "UniProtKB:Q9NX45",
  "term_id": "GO:0000981"
}